root hair cell differentiation [GO:0048765] (biological process) Definition: The process in which a relatively unspecialized cell acquires specialized features of a root hair cell. Sources: GOC:jid Relationships: is_a GO:0010053; is a type of GO:0048764